{
  "term_id": "UNKNOWN:0001",
  "gene_name": "EP300-interacting inhibitor of differentiation 3",
  "term_label": "Unknown molecular function",
  "gene": "UniProtKB:Q8N140",
  "gene_symbol": "EID3"
}